{
  "term_label": "protein serine/threonine kinase activity",
  "gene_symbol": "NUAK2",
  "gene_name": "NUAK family SNF1-like kinase 2",
  "gene": "UniProtKB:Q9H093",
  "term_id": "GO:0004674"
}